{
  "gene": "UniProtKB:Q5VT79",
  "gene_symbol": "ANXA8L1",
  "term_label": "endosome organization",
  "gene_name": "Annexin A8-like protein 1",
  "term_id": "GO:0007032"
}